negative regulation of receptor guanylyl cyclase signaling pathway [GO:0010754] (biological process) Definition: Any process that decreases the rate, frequency or extent of receptor guanylyl cyclase signaling pathway. References: PMID:24015261 Also known as: negative regulation of cGMP-mediated signaling, negative regulation of cGMP-mediated signalling Relationships: is a type of negative regulation of signal transduction [GO:0009968]; negatively regulates receptor guanylyl cyclase signaling pathway [GO:0007168]